cellular response to hydrogen sulfide [GO:1904881] (biological process) Definition: Any process that results in a change in state or activity of a cell (in terms of movement, secretion, enzyme production, gene expression, etc.) as a result of a hydrogen sulfide stimulus. References: PMID:24012591 Sources: GOC:TermGenie, GO_REF:0000071 Also known as: cellular response to dihydridosulfur, cellular response to sulfane Relationships: is a type of cellular response to chemical stimulus [GO:0070887]; is a type of GO:1904880